{
  "term_label": "cytosol",
  "gene_name": "DnaJ homolog subfamily B member 13",
  "gene_symbol": "DNAJB13",
  "gene": "UniProtKB:P59910",
  "term_id": "GO:0005829"
}